{
  "gene_symbol": "UMODL1",
  "term_id": "GO:0005615",
  "gene": "UniProtKB:Q5DID0",
  "term_label": "extracellular space",
  "gene_name": "Uromodulin-like 1"
}